{
  "term_label": "GID complex",
  "gene": "UniProtKB:Q9H871",
  "gene_symbol": "RMND5A",
  "gene_name": "E3 ubiquitin-protein transferase RMND5A",
  "term_id": "GO:0034657"
}